{
  "gene_symbol": "NDUFC2",
  "gene": "UniProtKB:O95298",
  "term_label": "Unknown biological process",
  "term_id": "UNKNOWN:0002",
  "gene_name": "NADH dehydrogenase [ubiquinone] 1 subunit C2"
}